{
  "term_label": "heterophilic cell-cell adhesion",
  "gene": "UniProtKB:Q86SJ2",
  "term_id": "GO:0007157",
  "gene_symbol": "AMIGO2",
  "gene_name": "Amphoterin-induced protein 2"
}